{
  "gene": "UniProtKB:Q4V326",
  "term_label": "Unknown biological process",
  "gene_symbol": "GAGE2E",
  "gene_name": "G antigen 2E",
  "term_id": "UNKNOWN:0002"
}